dorsal/ventral axis specification [GO:0009950] (biological process) Definition: The establishment, maintenance and elaboration of the dorsal/ventral axis. The dorsal/ventral axis is defined by a line that runs orthogonal to both the anterior/posterior and left/right axes. The dorsal end is defined by the upper or back side of an organism. The ventral end is defined by the lower or front side of an organism. Relationships: is a type of GO:0009798; is part of dorsal/ventral pattern formation [GO:0009953] Sources: GOC:dph, GOC:go_curators, GOC:tb Subtypes: oocyte dorsal/ventral axis specification [GO:0007310], GO:0007352, dorsal/ventral axis specification, ovarian follicular epithelium [GO:0008069] Also known as: dorsal-ventral axis specification, dorsoventral axis specification, dorsal/ventral axis determination